positive regulation of plant epidermal cell differentiation [GO:1903890] (biological process) Also known as: up regulation of plant epidermal cell differentiation, up-regulation of plant epidermal cell differentiation, upregulation of plant epidermal cell differentiation, activation of plant epidermal cell differentiation Definition: Any process that activates or increases the frequency, rate or extent of plant epidermal cell differentiation. Subtypes: GO:0010059, positive regulation of trichoblast fate specification [GO:0010063] References: PMID:123345 Sources: GOC:TermGenie, GO_REF:0000058 Relationships: is a type of positive regulation of cell differentiation [GO:0045597]; is a type of regulation of plant epidermal cell differentiation [GO:1903888]; positively regulates GO:0090627